{
  "gene_name": "Coatomer subunit alpha",
  "term_id": "GO:0006886",
  "gene": "UniProtKB:P53621",
  "term_label": "intracellular protein transport",
  "gene_symbol": "COPA"
}